{
  "term_id": "UNKNOWN:0003",
  "gene_symbol": "C2orf16",
  "gene_name": "Uncharacterized protein C2orf16",
  "term_label": "Unknown cellular component",
  "gene": "UniProtKB:Q68DN1"
}